{
  "term_label": "protein-folding chaperone binding",
  "gene_symbol": "DNAJB13",
  "gene_name": "DnaJ homolog subfamily B member 13",
  "gene": "UniProtKB:P59910",
  "term_id": "GO:0051087"
}